{
  "gene": "UniProtKB:Q96N95",
  "gene_symbol": "ZNF396",
  "term_id": "UNKNOWN:0003",
  "term_label": "Unknown cellular component",
  "gene_name": "Zinc finger protein 396"
}